{
  "gene": "UniProtKB:O95716",
  "term_label": "exocytosis",
  "gene_name": "Ras-related protein Rab-3D",
  "gene_symbol": "RAB3D",
  "term_id": "GO:0006887"
}